somatostatin receptor activity [GO:0004994] (molecular function) Definition: Combining with somatostatin to initiate a change in cell activity. Somatostatin is a peptide hormone that regulates the endocrine system by signaling via G protein-coupled somatostatin receptors. Somatostatin has two active forms produced by proteolytic cleavage: a 14 amino acid peptide (SST-14) and a 28 amino acid peptide (SST-28). Also known as: GHIH receptor activity, SRIF receptor activity, SST receptor activity, growth hormone-inhibiting hormone receptor activity, somatotrophin release inhibiting factor receptor activity Sources: GOC:ai, GOC:bf, Wikipedia:Somatostatin Relationships: is a type of neuropeptide receptor activity [GO:0008188]; is part of GO:0038170